adenosylcobinamide-phosphate synthase activity [GO:0043757] (molecular function) Sources: EC:6.3.1.10 Relationships: is_a acid-ammonia (or amide) ligase activity [GO:0016880] Also known as: adenosylcobyric acid:(R)-1-aminopropan-2-yl phosphate ligase (ADP-forming), AdoCbi-P synthase activity, CbiB Definition: Catalysis of the reactions: ATP + adenosylcobyric acid + (R)-1-aminopropan-2-yl phosphate = ADP + phosphate + adenosylcobinamide phosphate, and ATP + adenosylcobyric acid + (R)-1-aminopropan-2-ol = ADP + phosphate + adenosylcobinamide.